{
  "term_id": "GO:0004715",
  "gene_symbol": "ITK",
  "gene": "UniProtKB:Q08881",
  "term_label": "non-membrane spanning protein tyrosine kinase activity",
  "gene_name": "Tyrosine-protein kinase ITK_TSK"
}